{
  "term_id": "GO:0005886",
  "gene": "UniProtKB:Q6UY18",
  "gene_symbol": "LINGO4",
  "gene_name": "Leucine-rich repeat and immunoglobulin-like domain-containing nogo receptor-interacting protein 4",
  "term_label": "plasma membrane"
}